{
  "term_id": "UNKNOWN:0001",
  "gene_name": "Jouberin",
  "gene": "UniProtKB:Q8N157",
  "gene_symbol": "AHI1",
  "term_label": "Unknown molecular function"
}